{
  "term_id": "UNKNOWN:0003",
  "gene_symbol": "PPP1R2B",
  "gene_name": "Protein phosphatase inhibitor 2 family member B",
  "gene": "UniProtKB:Q6NXS1",
  "term_label": "Unknown cellular component"
}